{
  "gene_symbol": "HTR7",
  "term_label": "G protein-coupled serotonin receptor activity",
  "term_id": "GO:0004993",
  "gene": "UniProtKB:P34969",
  "gene_name": "5-hydroxytryptamine receptor 7"
}